multivesicular body, internal vesicle [GO:0097487] (CC) Relationships: is_a cytoplasmic vesicle [GO:0031410]; is part of multivesicular body [GO:0005771] Definition: A membrane-bounded vesicle wholly contained within a multivesicular body. References: PMID:21183070 Sources: GOC:pde